{
  "gene_name": "Protein ripply1",
  "gene_symbol": "RIPPLY1",
  "gene": "UniProtKB:Q0D2K3",
  "term_label": "Unknown molecular function",
  "term_id": "UNKNOWN:0001"
}